phosphoglycerate kinase (GTP) activity [GO:0050191] (molecular function) Sources: EC:2.7.2.10, RHEA:23332 Definition: Catalysis of the reaction: 3-phospho-D-glycerate + GTP = 3-phospho-D-glyceroyl phosphate + GDP + H+. Also known as: GTP:3-phospho-D-glycerate 1-phosphotransferase activity Relationships: is a type of kinase activity [GO:0016301]; is a type of GO:0016774